{
  "gene_symbol": "MICAL1",
  "term_label": "actin filament bundle assembly",
  "term_id": "GO:0051017",
  "gene_name": "[F-actin]-monooxygenase MICAL1",
  "gene": "UniProtKB:Q8TDZ2"
}